{
  "gene_name": "Olfactory receptor 10K2",
  "gene_symbol": "OR10K2",
  "gene": "UniProtKB:Q6IF99",
  "term_id": "GO:0005549",
  "term_label": "odorant binding"
}